cell septum [GO:0030428] (cellular component) Sources: GOC:clt, ISBN:0471940526 Relationships: is a type of cellular anatomical structure [GO:0110165] Also known as: septum, cross wall Subtypes: GO:0000933, porous cell septum [GO:0000934], division septum [GO:0000935] Definition: A structure composed of peptidoglycan and often chitin in addition to other materials. It usually forms perpendicular to the long axis of a cell or hypha and grows centripetally from the cell wall to the center of the cell and often functions in the compartmentalization of a cell into two daughter cells.